coronary vasculature morphogenesis [GO:0060977] (biological process) Relationships: is a type of GO:0048514; is part of coronary vasculature development [GO:0060976] Also known as: cardiac blood vessel morphogenesis, cardiac vasculature morphogenesis, coronary blood vessel morphogenesis, heart blood vessel morphogenesis, heart vasculature morphogenesis Sources: GOC:mtg_heart Subtypes: coronary vein morphogenesis [GO:0003169], coronary artery morphogenesis [GO:0060982] Definition: The process in which the anatomical structures of blood vessels of the heart are generated and organized. The blood vessel is the vasculature carrying blood.